{
  "term_id": "GO:0016567",
  "term_label": "protein ubiquitination",
  "gene_name": "Ubiquitin-like modifier-activating enzyme 6",
  "gene_symbol": "UBA6",
  "gene": "UniProtKB:A0AVT1"
}